{
  "gene_symbol": "ARGLU1",
  "gene": "UniProtKB:Q9NWB6",
  "gene_name": "Arginine and glutamate-rich protein 1",
  "term_id": "GO:0005739",
  "term_label": "mitochondrion"
}